peptide alpha-N-propionyltransferase activity [GO:0061607] (molecular function) References: PMID:23043182 Sources: GOC:dph Definition: Catalysis of the reaction: propionyl-CoA + peptide = CoA + N-alpha-propionylpeptide. This reaction is the propionylation of the N-terminal amino acid residue of a peptide or protein. Relationships: is a type of acyltransferase activity, transferring groups other than amino-acyl groups [GO:0016747]; is a type of catalytic activity, acting on a protein [GO:0140096]; is part of N-terminal protein amino acid propionylation [GO:0061606] Also known as: N-terminal propionyltransferase activity